farnesyl diphosphate biosynthetic process [GO:0045337] (biological process) Subtypes: farnesyl diphosphate biosynthetic process, mevalonate pathway [GO:0010142] Definition: The chemical reactions and pathways resulting in the formation of farnesyl diphosphate. Sources: GOC:jl Also known as: farnesyl diphosphate anabolism, farnesyl diphosphate biosynthesis, farnesyl diphosphate formation, farnesyl diphosphate synthesis Relationships: is_a GO:0008654; is a type of terpenoid biosynthetic process [GO:0016114]; is a type of farnesyl diphosphate metabolic process [GO:0045338]